{
  "term_id": "GO:0005794",
  "term_label": "Golgi apparatus",
  "gene_symbol": "ZDHHC15",
  "gene_name": "Palmitoyltransferase ZDHHC15",
  "gene": "UniProtKB:Q96MV8"
}